{
  "term_label": "Unknown molecular function",
  "term_id": "UNKNOWN:0001",
  "gene_symbol": "PSMB3",
  "gene_name": "Proteasome subunit beta type-3",
  "gene": "UniProtKB:P49720"
}